{
  "gene": "UniProtKB:Q9P275",
  "gene_symbol": "USP36",
  "gene_name": "Ubiquitin carboxyl-terminal hydrolase 36",
  "term_id": "GO:0005829",
  "term_label": "cytosol"
}